{
  "gene": "UniProtKB:P18054",
  "term_label": "cytosol",
  "gene_name": "Polyunsaturated fatty acid lipoxygenase ALOX12",
  "term_id": "GO:0005829",
  "gene_symbol": "ALOX12"
}